{
  "term_id": "GO:0000027",
  "term_label": "ribosomal large subunit assembly",
  "gene": "UniProtKB:Q9NZM5",
  "gene_name": "Ribosome biogenesis protein NOP53",
  "gene_symbol": "NOP53"
}